endosome lumen [GO:0031904] (CC) Subtypes: GO:0031905, late endosome lumen [GO:0031906], recycling endosome lumen [GO:0034777], endolysosome lumen [GO:0036021] Sources: GOC:mah Definition: The volume enclosed by the membrane of an endosome. Relationships: is a type of intracellular organelle lumen [GO:0070013]; is part of endosome [GO:0005768]